{
  "term_id": "GO:0045095",
  "gene_symbol": "KRT84",
  "gene": "UniProtKB:Q9NSB2",
  "gene_name": "Keratin, type II cuticular Hb4",
  "term_label": "keratin filament"
}